{
  "term_label": "cytokine activity",
  "gene": "UniProtKB:Q9NZH6",
  "term_id": "GO:0005125",
  "gene_name": "Interleukin-37",
  "gene_symbol": "IL37"
}